{
  "term_label": "G protein-coupled ATP receptor activity",
  "gene_name": "P2Y purinoceptor 11",
  "gene": "UniProtKB:Q96G91",
  "term_id": "GO:0045031",
  "gene_symbol": "P2RY11"
}